D-fructuronate reductase activity [GO:0102501] (molecular function) Definition: Catalysis of the reaction: D-mannonate + NADP = NADPH + H+ + D-fructuronate. Relationships: is a type of GO:0016616 References: PMID:22925190 Sources: GOC:pz